calcium activated phosphatidylserine scrambling [GO:0061589] (biological process) References: PMID:23532839 Sources: GOC:krc Definition: The movement of a population of phosphatidylserine molecules from one leaflet of the plasma membrane bilayer to the opposite leaflet as a result of a calcium stimulus. Relationships: is a type of calcium activated phospholipid scrambling [GO:0061588]